nucleolar ribonuclease P complex [GO:0005655] (cellular component) Also known as: nucleolar RNase P complex Definition: A ribonuclease P complex located in the nucleolus of a eukaryotic cell, where it catalyzes the 5' endonucleolytic cleavage of precursor tRNAs to yield mature tRNAs. Eukaryotic nucleolar ribonuclease P complexes generally contain a single RNA molecule that is necessary but not sufficient for catalysis, and several protein molecules. References: PMID:12045094 Sources: GOC:mah Relationships: is a type of multimeric ribonuclease P complex [GO:0030681]; is a type of nuclear protein-containing complex [GO:0140513]; is part of nucleolus [GO:0005730]